{
  "gene": "UniProtKB:P21281",
  "gene_name": "V-type proton ATPase subunit B, brain isoform",
  "gene_symbol": "ATP6V1B2",
  "term_label": "plasma membrane",
  "term_id": "GO:0005886"
}